{
  "gene": "UniProtKB:Q7L8C5",
  "term_label": "dense core granule",
  "term_id": "GO:0031045",
  "gene_name": "Synaptotagmin-13",
  "gene_symbol": "SYT13"
}